nuclear proteasome regulatory particle [GO:0031598] (cellular component) Sources: GOC:mah Relationships: is a type of proteasome regulatory particle [GO:0005838]; is a type of nuclear protein-containing complex [GO:0140513]; is part of nuclear proteasome complex [GO:0031595] Definition: The regulatory subcomplex of a proteasome located in the nucleus of a cell.